{
  "term_label": "Unknown biological process",
  "term_id": "UNKNOWN:0002",
  "gene_symbol": "TSPY3",
  "gene_name": "Testis-specific Y-encoded protein 3",
  "gene": "UniProtKB:P0CV98"
}